{
  "gene_name": "COMM domain-containing protein 5",
  "term_label": "Unknown molecular function",
  "gene": "UniProtKB:Q9GZQ3",
  "term_id": "UNKNOWN:0001",
  "gene_symbol": "COMMD5"
}